{
  "gene": "UniProtKB:Q13402",
  "term_id": "GO:0015629",
  "term_label": "actin cytoskeleton",
  "gene_name": "Unconventional myosin-VIIa",
  "gene_symbol": "MYO7A"
}